{
  "gene_name": "Solute carrier family 2, facilitated glucose transporter member 10",
  "gene_symbol": "SLC2A10",
  "term_label": "D-glucose transmembrane transporter activity",
  "gene": "UniProtKB:O95528",
  "term_id": "GO:0055056"
}